{
  "term_id": "GO:0033270",
  "gene": "UniProtKB:Q8TAM6",
  "gene_symbol": "ERMN",
  "gene_name": "Ermin",
  "term_label": "paranode region of axon"
}